plasma membrane fusion involved in cytogamy [GO:0032220] (biological process) Relationships: is a type of GO:0045026; is part of cytogamy [GO:0000755] References: PMID:29134248 Sources: GOC:mah Also known as: plasma membrane organization involved in conjugation with cellular fusion, plasma membrane fusion during cytogamy Definition: The joining of two or more lipid bilayer membranes that surround cells, that contributes to cytogamy.